{
  "gene_name": "Proteasome adapter and scaffold protein ECM29",
  "term_id": "GO:0005737",
  "term_label": "cytoplasm",
  "gene_symbol": "ECPAS",
  "gene": "UniProtKB:Q5VYK3"
}